{
  "gene_symbol": "MTHFR",
  "gene_name": "Methylenetetrahydrofolate reductase (NADPH)",
  "gene": "UniProtKB:P42898",
  "term_label": "cytosol",
  "term_id": "GO:0005829"
}